{
  "gene": "UniProtKB:Q99719",
  "term_label": "cytoskeleton-dependent cytokinesis",
  "term_id": "GO:0061640",
  "gene_name": "Septin-5",
  "gene_symbol": "SEPTIN5"
}